cell adhesion involved in single-species biofilm formation [GO:0043709] (BP) Regulation: regulated by regulation of cell adhesion involved in single-species biofilm formation [GO:1900187]; negatively regulated by negative regulation of cell adhesion involved in single-species biofilm formation [GO:1900188]; positively regulated by GO:1900189 Also known as: cell adhesion during single-species biofilm formation Relationships: is a type of cell adhesion involved in biofilm formation [GO:0043708]; is part of GO:0090609 Subtypes: cell adhesion involved in single-species biofilm formation in or on host organism [GO:0043707] Definition: The attachment of a cell to a solid substrate, via cell adhesion molecules, during the formation of a biofilm composed of microorganisms of the same species. Sources: GOC:dph, GOC:jl, GOC:tb